{
  "gene_name": "A-kinase anchor protein 8",
  "term_label": "nucleus",
  "term_id": "GO:0005634",
  "gene": "UniProtKB:O43823",
  "gene_symbol": "AKAP8"
}